{
  "gene_name": "Oxygen-regulated protein 1",
  "term_id": "GO:0035082",
  "gene_symbol": "RP1",
  "term_label": "axoneme assembly",
  "gene": "UniProtKB:P56715"
}